{
  "term_label": "cytosol",
  "term_id": "GO:0005829",
  "gene": "UniProtKB:P31944",
  "gene_name": "Caspase-14",
  "gene_symbol": "CASP14"
}